{
  "gene_symbol": "KIF2C",
  "gene_name": "Kinesin-like protein KIF2C",
  "term_id": "GO:0003777",
  "term_label": "microtubule motor activity",
  "gene": "UniProtKB:Q99661"
}